{
  "gene": "UniProtKB:A0A075B6N4",
  "term_id": "GO:0005886",
  "gene_name": "T cell receptor beta variable 25-1",
  "gene_symbol": "TRBV25-1",
  "term_label": "plasma membrane"
}